{
  "term_id": "GO:0005634",
  "gene": "UniProtKB:Q15742",
  "gene_symbol": "NAB2",
  "term_label": "nucleus",
  "gene_name": "NGFI-A-binding protein 2"
}